{
  "gene": "UniProtKB:O75419",
  "term_label": "DNA replication origin binding",
  "gene_symbol": "CDC45",
  "gene_name": "Cell division control protein 45 homolog",
  "term_id": "GO:0003688"
}